{
  "term_id": "GO:0035556",
  "gene_symbol": "PAK1",
  "gene_name": "Serine_threonine-protein kinase PAK 1",
  "gene": "UniProtKB:Q13153",
  "term_label": "intracellular signal transduction"
}